{
  "gene": "UniProtKB:P04798",
  "term_label": "toxin metabolic process",
  "gene_name": "Cytochrome P450 1A1",
  "gene_symbol": "CYP1A1",
  "term_id": "GO:0009404"
}